{
  "gene_name": "Cadherin-17",
  "term_id": "GO:0008013",
  "gene": "UniProtKB:Q12864",
  "term_label": "beta-catenin binding",
  "gene_symbol": "CDH17"
}